{
  "term_label": "histone H3K4 methyltransferase activity",
  "gene_name": "Actin-histidine N-methyltransferase",
  "gene_symbol": "SETD3",
  "gene": "UniProtKB:Q86TU7",
  "term_id": "GO:0042800"
}